semicircular canal morphogenesis [GO:0048752] (biological process) Also known as: embryonic semicircular canal morphogenesis Relationships: is a type of tube morphogenesis [GO:0035239]; is a type of GO:0048598; is part of inner ear morphogenesis [GO:0042472]; BFO_0000050 semicircular canal development [GO:0060872] Definition: The process in which the anatomical structures of the semicircular canals are generated and organized. Sources: GOC:dgh, GOC:dph, GOC:jid